{
  "term_label": "negative regulation of coagulation",
  "gene_symbol": "PROCR",
  "term_id": "GO:0050819",
  "gene": "UniProtKB:Q9UNN8",
  "gene_name": "Endothelial protein C receptor"
}